fungal-type cell wall beta-glucan biosynthetic process [GO:0070880] (biological process) Subtypes: GO:0034412, fungal-type cell wall (1->3)-beta-D-glucan biosynthetic process [GO:0071970] Sources: GOC:mah Also known as: fungal-type cell wall beta-glucan anabolism, fungal-type cell wall beta-glucan biosynthesis, fungal-type cell wall beta-glucan formation, fungal-type cell wall beta-glucan synthesis Definition: The chemical reactions and pathways resulting in the formation of beta-glucans, compounds composed of glucose residues linked by beta-D-glucosidic bonds, found in the walls of fungal cells. Regulation: regulated by regulation of fungal-type cell wall beta-glucan biosynthetic process [GO:0090093] Relationships: is a type of cell wall beta-glucan biosynthetic process [GO:0034410]; is a type of fungal-type cell wall polysaccharide biosynthetic process [GO:0051278]; is a type of fungal-type cell wall beta-glucan metabolic process [GO:0070879]